{
  "gene_name": "Double-strand-break repair protein rad21 homolog",
  "gene_symbol": "RAD21",
  "term_id": "GO:0030893",
  "term_label": "meiotic cohesin complex",
  "gene": "UniProtKB:O60216"
}